cyclopentanol dehydrogenase activity [GO:0055041] (MF) Also known as: cyclopentanol:NAD+ oxidoreductase activity, cyclopentanol:NADP+ oxidoreductase activity Definition: Catalysis of the reaction: cyclopentanol + NAD+ = cyclopentanone + H+ + NADH. Relationships: is a type of oxidoreductase activity, acting on the CH-OH group of donors, NAD or NADP as acceptor [GO:0016616] Sources: EC:1.1.1.163, RHEA:11728